{
  "gene_symbol": "RRP7A",
  "term_label": "Unknown molecular function",
  "term_id": "UNKNOWN:0001",
  "gene_name": "Ribosomal RNA-processing protein 7 homolog A",
  "gene": "UniProtKB:Q9Y3A4"
}